{
  "term_id": "GO:0015862",
  "gene_name": "Equilibrative nucleoside transporter 1",
  "gene": "UniProtKB:Q99808",
  "term_label": "uridine transmembrane transport",
  "gene_symbol": "SLC29A1"
}